{
  "gene_symbol": "CCDC17",
  "gene": "UniProtKB:Q96LX7",
  "term_label": "Unknown cellular component",
  "term_id": "UNKNOWN:0003",
  "gene_name": "Coiled-coil domain-containing protein 17"
}